{
  "gene": "UniProtKB:O75367",
  "term_id": "GO:0030527",
  "gene_symbol": "MACROH2A1",
  "gene_name": "Core histone macro-H2A.1",
  "term_label": "structural constituent of chromatin"
}